L-sorbose catabolic process [GO:0042850] (biological process) Definition: The chemical reactions and pathways resulting in the breakdown of L-sorbose, the L-enantiomer of the ketohexose xylo-2-hexulose. Relationships: is a type of GO:0019320 Sources: GOC:jsg, GOC:mah, ISBN:0198506732 Also known as: L-sorbose breakdown, L-sorbose catabolism, L-sorbose degradation